{
  "gene": "UniProtKB:Q03393",
  "term_id": "GO:0006729",
  "gene_name": "6-pyruvoyl tetrahydrobiopterin synthase",
  "term_label": "tetrahydrobiopterin biosynthetic process",
  "gene_symbol": "PTS"
}